{
  "gene_symbol": "BAIAP3",
  "gene": "UniProtKB:O94812",
  "gene_name": "BAI1-associated protein 3",
  "term_label": "plasma membrane",
  "term_id": "GO:0005886"
}